serine-type D-Ala-D-Ala carboxypeptidase activity [GO:0009002] (molecular function) Sources: EC:3.4.16.4 Also known as: D-alanine carboxypeptidase, DD-carboxypeptidase, D-alanyl carboxypeptidase activity, D-alanyl-D-alanine carboxypeptidase activity, D-alanyl-D-alanine-carboxypeptidase activity, D-alanyl-D-alanine-cleaving peptidase activity, D-alanyl-D-alanine-cleaving-peptidase activity, DD-peptidase activity, DD-transpeptidase activity Definition: Catalysis of the reaction: (Ac)2-L-Lys-D-alanyl-D-alanine + H2O = (Ac)2-L-Lys-D-alanine + D-alanine. Relationships: is a type of GO:0004185